regulation of arugosin biosynthetic process [GO:1900626] (biological process) Definition: Any process that modulates the frequency, rate or extent of arugosin biosynthetic process. Subtypes: GO:1900627, GO:1900628 Also known as: regulation of arugosin anabolism, regulation of arugosin biosynthesis, regulation of arugosin formation, regulation of arugosin synthesis Sources: GOC:TermGenie, GOC:di Relationships: is a type of regulation of secondary metabolite biosynthetic process [GO:1900376]; regulates arugosin biosynthetic process [GO:1900587]